{
  "gene_symbol": "LRP1",
  "gene": "UniProtKB:Q07954",
  "gene_name": "Prolow-density lipoprotein receptor-related protein 1",
  "term_label": "phagocytosis",
  "term_id": "GO:0006909"
}